{
  "gene_name": "Large ribosomal subunit protein uL4",
  "gene_symbol": "RPL4",
  "term_label": "cytosolic large ribosomal subunit",
  "gene": "UniProtKB:P36578",
  "term_id": "GO:0022625"
}